{
  "term_label": "cellular response to cAMP",
  "gene_name": "Ras-related protein Rap-1b-like protein",
  "term_id": "GO:0071320",
  "gene_symbol": "RAP1BL",
  "gene": "UniProtKB:A6NIZ1"
}